{
  "gene_symbol": "IGHD3-10",
  "gene": "UniProtKB:A0A0J9YXN1",
  "term_id": "UNKNOWN:0002",
  "term_label": "Unknown biological process",
  "gene_name": "Immunoglobulin heavy diversity 3-10 (Fragment)"
}